{
  "gene_name": "Glycine cleavage system H protein, mitochondrial",
  "term_id": "GO:0005739",
  "gene": "UniProtKB:P23434",
  "gene_symbol": "GCSH",
  "term_label": "mitochondrion"
}